2'-hydroxydaidzein reductase activity [GO:0047525] (molecular function) Also known as: 2'-hydroxy-2,3-dihydrodaidzein:NADP+ 2'-oxidoreductase activity, 2'-hydroxydihydrodaidzein:NADP(+) 2'-oxidoreductase activity, 2'-hydroxydihydrodaidzein:NADP+ 2'-oxidoreductase activity, HDR activity, NADPH:2'-hydroxydaidzein oxidoreductase activity Sources: EC:1.3.1.51 Relationships: is a type of oxidoreductase activity, acting on the CH-CH group of donors, NAD or NADP as acceptor [GO:0016628] Definition: Catalysis of the reaction: 2'-hydroxydihydrodaidzein + NADP+ = 2'-hydroxydaidzein + NADPH + H+.